squalene cyclase activity [GO:0034072] (MF) References: PMID:18033581 Sources: GOC:cb Definition: Catalysis of the reaction: squalene = triterpene. Relationships: is a type of GO:0009975 Subtypes: tetrahymanol synthase activity [GO:0034073], squalene-hopene cyclase activity [GO:0051007]